subtype 3 bombesin receptor binding [GO:0031706] (molecular function) Relationships: is_a bombesin receptor binding [GO:0031705] Also known as: subtype 3 bombesin receptor ligand Definition: Binding to a subtype 3 bombesin receptor. Sources: GOC:mah, GOC:nln